{
  "gene_name": "Caspase-4",
  "gene": "UniProtKB:P49662",
  "term_label": "cytosol",
  "gene_symbol": "CASP4",
  "term_id": "GO:0005829"
}